negative regulation of purine nucleobase metabolic process [GO:0045982] (biological process) Sources: GOC:go_curators Definition: Any process that stops, prevents, or reduces the frequency, rate or extent of the chemical reactions and pathways involving purine nucleobases. Also known as: down regulation of purine base metabolic process, down-regulation of purine base metabolic process, downregulation of purine base metabolic process, negative regulation of purine base metabolic process, negative regulation of purine base metabolism, inhibition of purine base metabolic process Relationships: is a type of GO:0006141; is a type of negative regulation of nucleobase-containing compound metabolic process [GO:0045934]; is a type of GO:0062014; RO_0002212 purine nucleobase metabolic process [GO:0006144]